{
  "term_id": "GO:0004709",
  "term_label": "MAP kinase kinase kinase activity",
  "gene_name": "Mitogen-activated protein kinase kinase kinase 15",
  "gene": "UniProtKB:Q6ZN16",
  "gene_symbol": "MAP3K15"
}